{
  "term_label": "nuclear speck",
  "gene_name": "Serine_arginine-rich splicing factor 2",
  "gene_symbol": "SRSF2",
  "term_id": "GO:0016607",
  "gene": "UniProtKB:Q01130"
}